{
  "gene": "UniProtKB:Q0VD86",
  "term_label": "cyclin-dependent protein serine/threonine kinase inhibitor activity",
  "term_id": "GO:0004861",
  "gene_name": "Protein INCA1",
  "gene_symbol": "INCA1"
}